{
  "gene_symbol": "CRBN",
  "term_id": "GO:0060173",
  "gene": "UniProtKB:Q96SW2",
  "term_label": "limb development",
  "gene_name": "Protein cereblon"
}